immune response to tumor cell [GO:0002418] (biological process) Definition: An immune system process that functions in the response of an organism to a tumor cell. Relationships: is a type of response to tumor cell [GO:0002347]; is a type of GO:0006955 Subtypes: tolerance induction to tumor cell [GO:0002413], GO:0002423, GO:0002424 Regulation: regulated by regulation of immune response to tumor cell [GO:0002837]; negatively regulated by negative regulation of immune response to tumor cell [GO:0002838]; positively regulated by positive regulation of immune response to tumor cell [GO:0002839] References: PMID:16730260 Sources: GOC:add, ISBN:0781735149